cell-cell adhesion mediator activity [GO:0098632] (molecular function) Relationships: is_a cell adhesion mediator activity [GO:0098631]; is part of cell-cell adhesion [GO:0098609] Definition: The binding by a cell-adhesion protein on the cell surface to an extracellular matrix component, to mediate adhesion of the cell to another cell. Sources: Wikipedia:Cell_adhesion Subtypes: protein binding involved in heterotypic cell-cell adhesion [GO:0086080], cadherin binding involved in cell-cell adhesion [GO:0098641] Also known as: cell-cell adhesion molecule, protein binding involved in cell-cell adhesion